{
  "term_label": "antigen processing and presentation, exogenous lipid antigen via MHC class Ib",
  "gene": "UniProtKB:P29016",
  "gene_symbol": "CD1B",
  "term_id": "GO:0048007",
  "gene_name": "T-cell surface glycoprotein CD1b"
}